GDP-mannose mannosyl hydrolase activity [GO:0008727] (molecular function) Relationships: is a type of GO:0015923 Definition: Catalysis of the reaction: GDP-alpha-D-mannose + H2O = GDP + D-mannose + H+. Sources: MetaCyc:GDPMANMANHYDRO-RXN